{
  "term_id": "GO:0005615",
  "gene_symbol": "BMP8A",
  "gene_name": "Bone morphogenetic protein 8A",
  "gene": "UniProtKB:Q7Z5Y6",
  "term_label": "extracellular space"
}